{
  "gene_name": "Large ribosomal subunit protein mL43",
  "term_label": "structural constituent of ribosome",
  "gene": "UniProtKB:Q8N983",
  "gene_symbol": "MRPL43",
  "term_id": "GO:0003735"
}